{
  "gene_symbol": "KCNJ3",
  "term_id": "GO:1990573",
  "gene": "UniProtKB:P48549",
  "gene_name": "G protein-activated inward rectifier potassium channel 1",
  "term_label": "potassium ion import across plasma membrane"
}